{
  "gene": "UniProtKB:P35218",
  "gene_symbol": "CA5A",
  "term_label": "Unknown biological process",
  "term_id": "UNKNOWN:0002",
  "gene_name": "Carbonic anhydrase 5A, mitochondrial"
}